{
  "gene": "UniProtKB:Q9Y672",
  "gene_symbol": "ALG6",
  "term_id": "GO:0005789",
  "gene_name": "Dolichyl pyrophosphate Man9GlcNAc2 alpha-1,3-glucosyltransferase",
  "term_label": "endoplasmic reticulum membrane"
}